{
  "term_id": "GO:0005885",
  "term_label": "Arp2/3 protein complex",
  "gene_name": "Actin-related protein 2_3 complex subunit 1A",
  "gene": "UniProtKB:Q92747",
  "gene_symbol": "ARPC1A"
}